{
  "gene_name": "Spermatogenic leucine zipper protein 1",
  "gene_symbol": "SPZ1",
  "term_label": "Unknown biological process",
  "gene": "UniProtKB:Q9BXG8",
  "term_id": "UNKNOWN:0002"
}